positive regulation of toll-like receptor 7 signaling pathway [GO:0034157] (biological process) Also known as: positive regulation of TLR7 signaling pathway, positive regulation of toll-like receptor 7 signalling pathway Relationships: is a type of regulation of toll-like receptor 7 signaling pathway [GO:0034155]; is a type of positive regulation of pattern recognition receptor signaling pathway [GO:0062208]; is a type of positive regulation of intracellular signal transduction [GO:1902533]; positively regulates GO:0034154 References: PMID:16551253, PMID:17328678 Sources: GOC:add Definition: Any process that activates or increases the frequency, rate, or extent of toll-like receptor 7 signaling pathway.